formate-dihydrofolate ligase activity [GO:0047897] (molecular function) Also known as: dihydrofolate formyltransferase activity, formate:dihydrofolate ligase (ADP-forming), formyl dihydrofolate synthase activity Definition: Catalysis of the reaction: 7,8-dihydrofolate + ATP + formate = 10-formyldihydrofolate + ADP + H+ + phosphate. Relationships: is a type of ligase activity, forming carbon-nitrogen bonds [GO:0016879] Sources: EC:6.3.4.17, RHEA:24328